{
  "term_label": "positive regulation of transcription by RNA polymerase II",
  "gene_name": "Thyrotroph embryonic factor",
  "gene_symbol": "TEF",
  "gene": "UniProtKB:Q10587",
  "term_id": "GO:0045944"
}